retromer, cargo-selective complex [GO:0030906] (cellular component) Definition: The trimeric subcomplex of the retromer, believed to be closely associated with the membrane. This trimeric complex is responsible for recognizing and binding to cargo molecules. The complex comprises three Vps proteins in both yeast and mammalian cells: Vps35p, Vps29p, and Vps26p in yeast, and VPS35, VPS29 and VPS26A or VPS26B in mammals. References: PMID:11102511, PMID:26220253, PMID:9700157 Sources: GOC:bf Also known as: cargo-selective retromer subcomplex, retromer CSC, retromer complex, inner shell, retromer, CRC, retromer, cargo recognition complex Relationships: is a type of membrane protein complex [GO:0098796]; is part of retromer complex [GO:0030904]